{
  "gene": "UniProtKB:Q15916",
  "term_id": "GO:0005654",
  "term_label": "nucleoplasm",
  "gene_name": "Zinc finger and BTB domain-containing protein 6",
  "gene_symbol": "ZBTB6"
}